{
  "term_id": "GO:0006357",
  "gene_symbol": "STAT2",
  "gene_name": "Signal transducer and activator of transcription 2",
  "term_label": "regulation of transcription by RNA polymerase II",
  "gene": "UniProtKB:P52630"
}